{
  "term_id": "GO:0005737",
  "gene_name": "Zinc finger MYND domain-containing protein 19",
  "gene": "UniProtKB:Q96E35",
  "term_label": "cytoplasm",
  "gene_symbol": "ZMYND19"
}